regulation of lymphocyte anergy [GO:0002911] (biological process) Relationships: is a type of regulation of tolerance induction [GO:0002643]; regulates GO:0002249 Definition: Any process that modulates the frequency, rate, or extent of lymphocyte anergy. Sources: GOC:add Subtypes: regulation of T cell anergy [GO:0002667], regulation of B cell anergy [GO:0002670], negative regulation of lymphocyte anergy [GO:0002912], positive regulation of lymphocyte anergy [GO:0002913]